tenascin complex [GO:0090733] (cellular component) Relationships: is a type of GO:0098637; is part of extracellular matrix [GO:0031012] Definition: A extracellular matrix complex involved in cell adhesion and cell migration. Typically homotrimeric or homohexameric. In mammals, four complexes exist: Tenascin-C, Tenascin-N (also known as Tenascin-W), Tenascin-X and Tenascin-R. Note: An example is Tenascin-N (Q9UQP3) in PMID:17909022 (IDA). References: PMID:11731446, PMID:12845616, PMID:17909022, PMID:23658023 Sources: GOC:bhm Also known as: Tenascin-C, Tenascin-N, Tenascin-R, Tenascin-W, Tenascin-X